{
  "term_label": "nucleoplasm",
  "gene": "UniProtKB:Q9BSH3",
  "gene_symbol": "NICN1",
  "gene_name": "Nicolin-1",
  "term_id": "GO:0005654"
}